oxidised low-density lipoprotein particle receptor activity [GO:0150025] (molecular function) Also known as: ox-LDL particle receptor activity, oxLDL particle receptor activity, oxidised LDL particle receptor activity, oxidized LDL particle receptor activity, oxidized low-density lipoprotein particle receptor activity, ox-LDL receptor activity, oxLDL receptor activity, oxidised LDL receptor activity, oxidised low-density lipoprotein receptor activity, oxidized LDL receptor activity, oxidized low-density lipoprotein receptor activity Relationships: is a type of lipoprotein particle receptor activity [GO:0030228] Definition: Combining with an oxidised low-density lipoprotein particle and delivering the oxidised low-density lipoprotein particle into the cell via endocytosis. References: PMID:27607416 Sources: GOC:aruk, GOC:bc